{
  "term_id": "GO:0005886",
  "term_label": "plasma membrane",
  "gene_name": "Cell cycle control protein 50B",
  "gene": "UniProtKB:Q3MIR4",
  "gene_symbol": "TMEM30B"
}